{
  "term_id": "GO:0030154",
  "gene_name": "Non-receptor tyrosine-protein kinase TYK2",
  "term_label": "cell differentiation",
  "gene_symbol": "TYK2",
  "gene": "UniProtKB:P29597"
}